positive regulation of protein localization to medial cortical node [GO:0120047] (biological process) Definition: Any process that activates or increases the frequency, rate or extent of protein localization to a medial cortical node. Relationships: is a type of positive regulation of protein localization to medial cortex [GO:0106012]; is a type of regulation of protein localization to medial cortical node [GO:0120046]; positively regulates protein localization to medial cortical node [GO:1902577] References: PMID:19474789